regulation of vitellogenesis [GO:1903186] (biological process) Subtypes: negative regulation of vitellogenesis [GO:1903187], GO:1903188 Also known as: regulation of yolk production Relationships: is a type of regulation of cellular component organization [GO:0051128]; is a type of regulation of multicellular organismal process [GO:0051239]; regulates GO:0007296 References: PMID:19467235 Sources: GOC:TermGenie, GOC:mr, GO_REF:0000058 Definition: Any process that modulates the frequency, rate or extent of vitellogenesis.